platelet dense tubular network lumen [GO:0031096] (cellular component) References: PMID:1322202 Sources: GOC:mah Relationships: is a type of intracellular organelle lumen [GO:0070013]; is part of platelet dense tubular network [GO:0031094] Definition: The volume enclosed by the membranes of the platelet dense tubular network.